light-harvesting complex, core complex [GO:0030078] (CC) Sources: GOC:lr Definition: Light harvesting complex associated with the reaction complex of photosynthetic purple bacteria. Relationships: is_a plasma membrane light-harvesting complex [GO:0030077]